macrolide 2'-kinase activity [GO:0050073] (molecular function) Also known as: ATP:macrolide 2'-O-phosphotransferase activity Sources: EC:2.7.1.136, RHEA:18333 Definition: Catalysis of the reaction: ATP + oleandomycin = ADP + 2 H+ + oleandomycin 2'-O-phosphate. Relationships: is a type of kinase activity [GO:0016301]; is a type of GO:0016773